calcium ion export across plasma membrane [GO:1990034] (biological process) References: PMID:2145281 Sources: GOC:mah Regulation: regulated by regulation of calcium ion export across plasma membrane [GO:1905912]; negatively regulated by GO:1905913; positively regulated by positive regulation of calcium ion export across plasma membrane [GO:1905914] Relationships: is a type of calcium ion transmembrane transport [GO:0070588]; is_a export across plasma membrane [GO:0140115] Definition: The directed movement of calcium ions from inside of a cell, across the plasma membrane and into the extracellular region. Also known as: calcium ion efflux from cell, calcium ion export from cell